{
  "term_id": "UNKNOWN:0003",
  "gene_symbol": "APOL4",
  "gene": "UniProtKB:Q9BPW4",
  "term_label": "Unknown cellular component",
  "gene_name": "Apolipoprotein L4"
}